{
  "gene_symbol": "ZBTB43",
  "term_label": "Unknown cellular component",
  "term_id": "UNKNOWN:0003",
  "gene": "UniProtKB:O43298",
  "gene_name": "Zinc finger and BTB domain-containing protein 43"
}